alpha9-beta1 integrin-ADAM1 complex [GO:0071052] (cellular component) Definition: A protein complex that consists of an alpha9-beta1 integrin complex bound to the transmembrane metallopeptidase ADAM1. References: PMID:11882657 Also known as: ITGA9-ITGB1-ADAM1 complex Relationships: is a type of plasma membrane protein complex [GO:0098797]